{
  "gene_name": "Fascin-2",
  "gene_symbol": "FSCN2",
  "term_id": "GO:0051017",
  "term_label": "actin filament bundle assembly",
  "gene": "UniProtKB:O14926"
}